DNA replication termination [GO:0006274] (biological process) References: PMID:10209736, PMID:12009298 Sources: GOC:mah Regulation: RO_0002211 by GO:2000621 Subtypes: site-specific DNA replication termination [GO:0071170], cell cycle DNA replication termination [GO:1902294] Relationships: is a type of GO:0006259; is part of DNA-templated DNA replication [GO:0006261] Definition: The process in which DNA replication at a replication fork ceases; occurs when the replication fork reaches a specific termination site or when two replication forks meet.